cellular response to water stimulus [GO:0071462] (biological process) Sources: GOC:mah Subtypes: cellular response to water deprivation [GO:0042631], GO:0071463, GO:0071464 Relationships: is a type of response to water [GO:0009415]; is a type of cellular response to abiotic stimulus [GO:0071214]; is a type of GO:0071229; is a type of GO:1901701 Definition: Any process that results in a change in state or activity of a cell (in terms of movement, secretion, enzyme production, gene expression, etc.) as a result of a stimulus reflecting the presence, absence, or concentration of water.